rRNA modification guide activity [GO:0030556] (molecular function) Subtypes: GO:0030559, GO:0030562 Note: Note that this term describes the activity of a nucleic acid, usually RNA, gene product that interacts with other RNA molecules via base pairing; it should not be used to annotate proteins. References: PMID:12457565 Sources: GOC:mah Relationships: is a type of rRNA binding [GO:0019843]; is a type of RNA modification guide activity [GO:0030555] Definition: Specifies the site of a posttranscriptional modification in an rRNA molecule by base pairing with a short sequence around the target residue.